{
  "term_id": "UNKNOWN:0001",
  "gene_symbol": "WDFY3",
  "gene": "UniProtKB:Q8IZQ1",
  "term_label": "Unknown molecular function",
  "gene_name": "WD repeat and FYVE domain-containing protein 3"
}